{
  "term_id": "UNKNOWN:0002",
  "gene_symbol": "MPHOSPH10",
  "term_label": "Unknown biological process",
  "gene_name": "U3 small nucleolar ribonucleoprotein protein MPP10",
  "gene": "UniProtKB:O00566"
}